translesion synthesis [GO:0019985] (BP) Also known as: bypass DNA synthesis References: PMID:10535901 Sources: GOC:elh, GOC:vw Subtypes: error-prone translesion synthesis [GO:0042276], error-free translesion synthesis [GO:0070987] Definition: The replication of damaged DNA by synthesis across a lesion in the template strand; a specialized DNA polymerase or replication complex inserts a defined nucleotide across from the lesion which allows DNA synthesis to continue beyond the lesion. This process can be mutagenic depending on the damaged nucleotide and the inserted nucleotide. Relationships: is a type of GO:0006301; is a type of DNA synthesis involved in DNA replication [GO:0090592]